{
  "term_label": "regulation of cell cycle",
  "gene": "UniProtKB:Q3YBR2",
  "gene_symbol": "TBRG1",
  "gene_name": "Transforming growth factor beta regulator 1",
  "term_id": "GO:0051726"
}